regulation of muscle hyperplasia [GO:0014738] (biological process) Definition: Any process that modulates the frequency, rate or extent of muscle hyperplasia. Sources: GOC:mtg_muscle Relationships: is a type of regulation of muscle adaptation [GO:0043502]; regulates muscle hyperplasia [GO:0014900] Subtypes: positive regulation of muscle hyperplasia [GO:0014739], GO:0014740, regulation of myofibril number [GO:0014882]